{
  "gene_name": "Large ribosomal subunit protein mL42",
  "term_id": "GO:0005762",
  "gene": "UniProtKB:Q9Y6G3",
  "gene_symbol": "MRPL42",
  "term_label": "mitochondrial large ribosomal subunit"
}